{
  "gene_symbol": "LGALS13",
  "gene": "UniProtKB:Q9UHV8",
  "term_label": "Unknown biological process",
  "term_id": "UNKNOWN:0002",
  "gene_name": "Galactoside-binding soluble lectin 13"
}